{
  "gene": "UniProtKB:Q9Y2X7",
  "gene_symbol": "GIT1",
  "term_label": "synaptic vesicle recycling",
  "gene_name": "ARF GTPase-activating protein GIT1",
  "term_id": "GO:0036465"
}